{
  "term_id": "UNKNOWN:0001",
  "gene_name": "Putative uncharacterized protein FLJ37218",
  "gene": "UniProtKB:Q8N1Y9",
  "term_label": "Unknown molecular function",
  "gene_symbol": "Q8N1Y9"
}